{
  "term_id": "GO:0036409",
  "term_label": "histone H3-K14 acetyltransferase complex",
  "gene_name": "Histone acetyltransferase KAT7",
  "gene": "UniProtKB:O95251",
  "gene_symbol": "KAT7"
}